{
  "gene_symbol": "KRTAP10-11",
  "term_id": "UNKNOWN:0003",
  "term_label": "Unknown cellular component",
  "gene": "UniProtKB:P60412",
  "gene_name": "Keratin-associated protein 10-11"
}